{
  "gene": "UniProtKB:Q13555",
  "term_id": "GO:0005737",
  "term_label": "cytoplasm",
  "gene_symbol": "CAMK2G",
  "gene_name": "Calcium_calmodulin-dependent protein kinase type II subunit gamma"
}